{
  "gene": "UniProtKB:Q9HBD1",
  "gene_name": "Roquin-2",
  "gene_symbol": "RC3H2",
  "term_label": "RNA stem-loop binding",
  "term_id": "GO:0035613"
}